{
  "gene_name": "Luc7-like protein 3",
  "gene_symbol": "LUC7L3",
  "term_label": "U2-type prespliceosome",
  "gene": "UniProtKB:O95232",
  "term_id": "GO:0071004"
}